regulation of central B cell deletion [GO:0002898] (biological process) Sources: GOC:add Definition: Any process that modulates the frequency, rate, or extent of central B cell deletion. Subtypes: GO:0002899, positive regulation of central B cell deletion [GO:0002900] Relationships: is_a regulation of B cell deletion [GO:0002867]; is a type of regulation of central B cell tolerance induction [GO:0002895]; is a type of regulation of B cell differentiation [GO:0045577]; regulates GO:0002342